{
  "gene_symbol": "CDON",
  "term_id": "GO:0098609",
  "gene": "UniProtKB:Q4KMG0",
  "term_label": "cell-cell adhesion",
  "gene_name": "Cell adhesion molecule-related_down-regulated by oncogenes"
}